{
  "gene": "UniProtKB:Q9NZL6",
  "gene_name": "Ral guanine nucleotide dissociation stimulator-like 1",
  "term_id": "GO:0005886",
  "term_label": "plasma membrane",
  "gene_symbol": "RGL1"
}